{
  "term_id": "GO:0015629",
  "gene_name": "Destrin",
  "gene": "UniProtKB:P60981",
  "term_label": "actin cytoskeleton",
  "gene_symbol": "DSTN"
}